{
  "term_id": "GO:0007165",
  "gene_name": "Fas apoptotic inhibitory molecule 3",
  "gene": "UniProtKB:O60667",
  "term_label": "signal transduction",
  "gene_symbol": "FCMR"
}